{
  "gene_symbol": "ORM2",
  "term_id": "GO:0005615",
  "gene": "UniProtKB:P19652",
  "term_label": "extracellular space",
  "gene_name": "Alpha-1-acid glycoprotein 2"
}